{
  "gene": "UniProtKB:Q13336",
  "term_id": "GO:0071918",
  "term_label": "urea transmembrane transport",
  "gene_name": "Urea transporter 1",
  "gene_symbol": "SLC14A1"
}